{
  "gene_name": "Putative peptide YY-3",
  "gene_symbol": "PYY3",
  "term_label": "feeding behavior",
  "term_id": "GO:0007631",
  "gene": "UniProtKB:Q5JQD4"
}